dTDP-galactose 6-dehydrogenase activity [GO:0033701] (molecular function) Also known as: dTDP-D-galactose:NADP+ 6-oxidoreductase activity, dTDPgalactose 6-dehydrogenase activity, thymidine-diphosphate-galactose dehydrogenase activity Definition: Catalysis of the reaction: dTDP-D-galactose + 2 NADP+ + H2O = dTDP-D-galacturonate + 2 NADPH + 2 H+. Sources: EC:1.1.1.186 Relationships: is a type of GO:0016616